{
  "term_label": "signal transduction",
  "gene_name": "Rho-related GTP-binding protein RhoU",
  "term_id": "GO:0007165",
  "gene_symbol": "RHOU",
  "gene": "UniProtKB:Q7L0Q8"
}